{
  "gene_symbol": "PRMT5",
  "gene": "UniProtKB:O14744",
  "term_id": "GO:0005634",
  "term_label": "nucleus",
  "gene_name": "Protein arginine N-methyltransferase 5"
}